vasoactive intestinal polypeptide receptor binding [GO:0031890] (molecular function) Relationships: is a type of neuropeptide receptor binding [GO:0071855] Sources: GOC:mah, GOC:nln Definition: Binding to a vasoactive intestinal polypeptide receptor. Also known as: VIP receptor binding, vasoactive intestinal polypeptide receptor ligand Subtypes: type 1 vasoactive intestinal polypeptide receptor binding [GO:0031891], type 2 vasoactive intestinal polypeptide receptor binding [GO:0031892]